{
  "term_label": "nucleus",
  "gene_symbol": "PRMT9",
  "gene_name": "Protein arginine N-methyltransferase 9",
  "term_id": "GO:0005634",
  "gene": "UniProtKB:Q6P2P2"
}